{
  "gene_name": "Forkhead box protein D4-like 4",
  "term_id": "UNKNOWN:0003",
  "gene_symbol": "FOXD4L4",
  "gene": "UniProtKB:Q8WXT5",
  "term_label": "Unknown cellular component"
}